{
  "gene_symbol": "OR6N2",
  "gene_name": "Olfactory receptor 6N2",
  "term_label": "membrane",
  "gene": "UniProtKB:Q8NGY6",
  "term_id": "GO:0016020"
}